{
  "term_id": "GO:0038187",
  "gene_symbol": "CLEC4E",
  "gene_name": "C-type lectin domain family 4 member E",
  "gene": "UniProtKB:Q9ULY5",
  "term_label": "pattern recognition receptor activity"
}